bradykinin receptor binding [GO:0031711] (molecular function) Relationships: is a type of G protein-coupled receptor binding [GO:0001664] Sources: GOC:mah, GOC:nln Subtypes: B1 bradykinin receptor binding [GO:0031712], B2 bradykinin receptor binding [GO:0031713] Also known as: bradykinin receptor ligand Definition: Binding to a bradykinin receptor.